{
  "term_label": "Unknown biological process",
  "gene_name": "Olfactory receptor 6J1",
  "gene": "UniProtKB:Q8NGC5",
  "gene_symbol": "OR6J1",
  "term_id": "UNKNOWN:0002"
}